{
  "term_label": "Unknown biological process",
  "gene_name": "Basic salivary proline-rich protein 1",
  "term_id": "UNKNOWN:0002",
  "gene": "UniProtKB:P04280",
  "gene_symbol": "PRB1"
}